{
  "term_label": "cytoplasm",
  "gene": "UniProtKB:O15111",
  "term_id": "GO:0005737",
  "gene_symbol": "CHUK",
  "gene_name": "Inhibitor of nuclear factor kappa-B kinase subunit alpha"
}